{
  "gene_symbol": "TUBA8",
  "term_label": "microtubule cytoskeleton organization",
  "gene": "UniProtKB:Q9NY65",
  "term_id": "GO:0000226",
  "gene_name": "Tubulin alpha-8 chain"
}